positive regulation of amyloid fibril formation [GO:1905908] (biological process) Definition: Any process that activates or increases the frequency, rate or extent of amyloid fibril formation. Also known as: up regulation of amyloid fibril formation, up-regulation of amyloid fibril formation, upregulation of amyloid fibril formation, activation of amyloid fibril formation, activation of amyloid fibril assembly, activation of amyloid structure assembly, activation of amyloid structure formation, positive regulation of amyloid fibril assembly, positive regulation of amyloid structure assembly, positive regulation of amyloid structure formation, up regulation of amyloid fibril assembly, up regulation of amyloid structure assembly, up regulation of amyloid structure formation, up-regulation of amyloid fibril assembly, up-regulation of amyloid structure assembly, up-regulation of amyloid structure formation, upregulation of amyloid fibril assembly, upregulation of amyloid structure assembly, upregulation of amyloid structure formation Relationships: is a type of positive regulation of protein metabolic process [GO:0051247]; is a type of positive regulation of supramolecular fiber organization [GO:1902905]; is a type of GO:1905906; RO_0002213 amyloid fibril formation [GO:1990000] Note: Although deposition of amyloid fibrils is associated with diseases, e.g. Alzheimer's disease, amyloid formation is a normal process. Disease occurs when the balance between amyloid formation and clearance is disrupted (reviewed e.g. in PMID:29654159 and PMID:28937655). An example of a normal amyloid complex is composed of human RIP1 and RIP3 kinases (PMID:22817896). References: PMID:23106396 Sources: GOC:TermGenie, GOC:aruk, GOC:bc, GO_REF:0000058